{
  "term_label": "vesicle fusion",
  "term_id": "GO:0006906",
  "gene_name": "Syntaxin-12",
  "gene": "UniProtKB:Q86Y82",
  "gene_symbol": "STX12"
}